venom-mediated activation of pH-gated ion channel activity [GO:0044734] (biological process) References: PMID:23034652 Sources: GOC:fj, GOC:jl Relationships: is a type of GO:0044733 Definition: A process in which an organism initiates, promotes, or enhances the activity of a pH-gated (also known as acid-sensing ion channel (ASIC)) in another organism via the action of a venom. Also known as: envenomation resulting in positive regulation of ASIC channel activity in other organism, envenomation resulting in positive regulation of acid-sensing ion channel activity in another organism, envenomation resulting in positive regulation of acid-sensing ion channel activity in other organism, venom-mediated activation of acid-sensing ion channel activity